phosphatidylethanolamine flippase activity [GO:0090555] (molecular function) Relationships: is a type of glycerophospholipid flippase activity [GO:0140333] Definition: Catalysis of the movement of phosphatidylethanolamine from the exoplasmic to the cytosolic leaflet of a membrane, using energy from the hydrolysis of ATP. References: PMID:16452632, PMID:20043909 Sources: GOC:ab Note: Nomenclature note. Flippases and floppases are ATP-dependent transbilayer lipid translocators. According to an extensively used, though not universal, nomenclature, they catalyze lipid transfer towards the inward monolayer (flippases) or towards the outward monolayer (floppases). Scramblases are ATP-independent, non-selective, inducing non-specific transbilayer movements across the membrane. The direction of the translocation should be taken into account for annotation (from the exoplasmic to the cytosolic leaflet of a membrane). Also known as: ATPase-coupled phosphatidylethanolamine transporter activity, phosphatidylethanolamine flippase activity (exoplasmic to cytosolic leaflet), ATP-dependent phosphatidylethanolamine transporter activity, phosphatidylethanolamine-translocating ATPase activity